{
  "term_label": "Unknown cellular component",
  "gene_symbol": "RNASEL",
  "term_id": "UNKNOWN:0003",
  "gene": "UniProtKB:Q05823",
  "gene_name": "2-5A-dependent ribonuclease"
}